halogen metabolic process [GO:0070276] (biological process) Definition: The chemical reactions and pathways involving any halogen, elements of Group VII; includes metabolism of halogen-containing compounds. Sources: GOC:mah Also known as: halogen metabolism Relationships: is a type of small molecule metabolic process [GO:0044281]